regulation of myeloid dendritic cell activation [GO:0030885] (biological process) Sources: GOC:mah Relationships: is a type of regulation of leukocyte activation [GO:0002694]; regulates GO:0001773 Subtypes: negative regulation of myeloid dendritic cell activation [GO:0030886], positive regulation of myeloid dendritic cell activation [GO:0030887] Definition: Any process that modulates the frequency or rate of myeloid dendritic cell activation.